plant-type vacuole membrane [GO:0009705] (cellular component) Definition: The lipid bilayer surrounding a vacuole that retains the same shape regardless of cell cycle phase. The membrane separates its contents from the cytoplasm of the cell. An example of this component is found in Arabidopsis thaliana. Sources: GOC:mtg_sensu, ISBN:0471245208 Also known as: vacuolar membrane, membrane of vacuole with cell cycle-independent morphology, tonoplast Relationships: is a type of GO:0005774; is part of GO:0000325 Subtypes: protein storage vacuole membrane [GO:0032586]